retrograde transport, vesicle recycling within Golgi [GO:0000301] (biological process) Also known as: retrograde (vesicle recycling within Golgi) transport Definition: The retrograde movement of substances within the Golgi, mediated by COP I vesicles. Cis-Golgi vesicles are constantly moving forward through the Golgi stack by cisternal progression, eventually becoming trans-Golgi vesicles. They then selectively transport membrane and luminal proteins from the trans- to the medial-Golgi while leaving others behind in the trans-Golgi cisternae; similarly, they selectively move proteins from the medial- to the cis-Golgi. Sources: ISBN:0716731363 Relationships: is a type of GO:0006891